positive regulation of embryo sac central cell differentiation [GO:0045693] (biological process) Definition: Any process that activates or increases the frequency, rate or extent of embryo sac central cell differentiation. Sources: GOC:go_curators, GOC:mtg_plant Also known as: positive regulation of female gametophyte central cell differentiation, up regulation of female gametophyte central cell differentiation, up-regulation of female gametophyte central cell differentiation, upregulation of female gametophyte central cell differentiation, activation of female gametophyte central cell differentiation, stimulation of female gametophyte central cell differentiation Relationships: is a type of positive regulation of cell differentiation [GO:0045597]; is a type of regulation of embryo sac central cell differentiation [GO:0045691]; is a type of positive regulation of multicellular organismal process [GO:0051240]; positively regulates embryo sac central cell differentiation [GO:0009559]